{
  "term_label": "nucleus",
  "gene_symbol": "SETDB2",
  "gene_name": "Histone-lysine N-methyltransferase SETDB2",
  "term_id": "GO:0005634",
  "gene": "UniProtKB:Q96T68"
}